{
  "gene_symbol": "A0A0G2JNJ9",
  "gene": "UniProtKB:A0A0G2JNJ9",
  "gene_name": "Uncharacterized protein",
  "term_id": "UNKNOWN:0003",
  "term_label": "Unknown cellular component"
}